1-aminocyclopropane-1-carboxylate synthase activity [GO:0016847] (molecular function) Relationships: is_a carbon-sulfur lyase activity [GO:0016846]; is part of 1-aminocyclopropane-1-carboxylate biosynthetic process [GO:0042218] Also known as: 1-aminocyclopropane-1-carboxylate synthetase activity, 1-aminocyclopropane-1-carboxylic acid synthase activity, 1-aminocyclopropanecarboxylate synthase activity, ACC synthase activity, L-VG deaminase activity, L-vinylglycine deaminase activity, S-adenosyl-L-methionine methylthioadenosine-lyase (1-aminocyclopropane-1-carboxylate-forming), S-adenosyl-L-methionine methylthioadenosine-lyase activity, aminocyclopropanecarboxylate synthase activity, aminocyclopropanecarboxylic acid synthase activity Sources: EC:4.4.1.14, RHEA:21744 Definition: Catalysis of the reaction: S-adenosyl-L-methionine(1+) = 1-aminocyclopropane-1-carboxylate + S-methyl-5'-thioadenosine + H+.